{
  "gene_name": "Protein HRURF",
  "gene": "UniProtKB:P0DUH7",
  "term_label": "Unknown molecular function",
  "term_id": "UNKNOWN:0001",
  "gene_symbol": "HRURF"
}